mitotic chromosome movement towards spindle pole [GO:0007079] (biological process) Also known as: mitotic chromosome movement, chromosome migration to spindle pole during mitosis, chromosome movement towards spindle pole during mitosis, mitotic chromosome movement to spindle pole, mitotic sister chromosome movement towards spindle pole, sister chromosome movement towards spindle pole during mitosis Sources: GOC:ai Relationships: is a type of GO:0051305; is a type of mitotic cell cycle process [GO:1903047]; is part of mitotic sister chromatid segregation [GO:0000070] Definition: The cell cycle process in which the directed movement of chromosomes from the center of the spindle towards the spindle poles occurs. This mediates by the shortening of microtubules attached to the chromosomes, during mitosis.